2-aminohexanoate transaminase activity [GO:0047537] (molecular function) Also known as: 2-aminohexanoate aminotransferase activity, L-2-aminohexanoate:2-oxoglutarate aminotransferase activity, leucine L-norleucine: 2-oxoglutarate aminotransferase activity, norleucine (leucine) aminotransferase activity, norleucine aminotransferase activity, norleucine transaminase activity Relationships: is a type of transaminase activity [GO:0008483] Sources: EC:2.6.1.67, MetaCyc:2-AMINOHEXANOATE-AMINOTRANSFERASE-RXN Definition: Catalysis of the reaction: L-2-aminohexanoate + 2-oxoglutarate = 2-oxohexanoate + L-glutamate.